negative regulation of thermomorphogenesis [GO:0140921] (biological process) Relationships: is a type of negative regulation of post-embryonic development [GO:0048581]; is_a GO:0048585; is a type of regulation of thermomorphogenesis [GO:0140920]; negatively regulates thermomorphogenesis [GO:0140919] Definition: Any process that stops, prevents or reduces the frequency, rate or extent of thermomorphogenesis. References: PMID:27250752